regulation of penile erection [GO:0060405] (biological process) Definition: Any process that modulates the rate, frequency or extent of penile erection. Penile erection is the hardening, enlarging and rising of the penis which often occurs in the sexually aroused male and enables sexual intercourse. Achieved by increased inflow of blood into the vessels of erectile tissue, and decreased outflow. Sources: GOC:add, GOC:dph, GOC:tb Relationships: is a type of regulation of multicellular organismal process [GO:0051239]; is a type of regulation of reproductive process [GO:2000241]; regulates GO:0043084 Subtypes: positive regulation of penile erection [GO:0060406], negative regulation of penile erection [GO:0060407]